{
  "gene_symbol": "C4orf47",
  "gene": "UniProtKB:A7E2U8",
  "term_id": "UNKNOWN:0001",
  "gene_name": "UPF0602 protein C4orf47",
  "term_label": "Unknown molecular function"
}